negative regulation of syncytial blastoderm mitotic cell cycle [GO:0046003] (biological process) Definition: Any process that stops, prevents or reduces the rate or extent of progression through the syncytial blastoderm mitotic cell cycle. Sources: GOC:dph, GOC:go_curators, GOC:tb Also known as: down regulation of progression through syncytial blastoderm mitotic cell cycle, down-regulation of progression through syncytial blastoderm mitotic cell cycle, downregulation of progression through syncytial blastoderm mitotic cell cycle, negative regulation of progression through syncytial blastoderm mitotic cell cycle, negative regulation of syncytial blastoderm cell cycle progression, inhibition of progression through syncytial blastoderm mitotic cell cycle Relationships: is a type of GO:0007348; is a type of GO:0045976; negatively regulates syncytial blastoderm mitotic cell cycle [GO:0035186]